maturation of 5S rRNA from tetracistronic rRNA transcript (SSU-rRNA, 5.8S rRNA, LSU-rRNA) [GO:0000482] (BP) Sources: GOC:curators Definition: Any process involved in the maturation of a precursor 5S ribosomal RNA (rRNA) molecule into a mature 5S rRNA molecule from the pre-rRNA molecule originally produced as a tetracistronic rRNA transcript that contains the Small Subunit (SSU) rRNA, Large Subunit (LSU) the 4.5S rRNA, and the 5S rRNA in that order from 5' to 3' along the primary transcript. Relationships: is a type of GO:0000481